{
  "term_id": "GO:0005737",
  "gene_name": "Annexin A11",
  "term_label": "cytoplasm",
  "gene_symbol": "ANXA11",
  "gene": "UniProtKB:P50995"
}